{
  "term_label": "axon guidance",
  "gene_name": "Kinesin-1 heavy chain",
  "gene": "UniProtKB:P33176",
  "gene_symbol": "KIF5B",
  "term_id": "GO:0007411"
}